{
  "gene_name": "Ras-related C3 botulinum toxin substrate 1",
  "term_label": "regulation of actin cytoskeleton organization",
  "gene_symbol": "RAC1",
  "term_id": "GO:0032956",
  "gene": "UniProtKB:P63000"
}